{
  "term_id": "GO:0015229",
  "gene_name": "Solute carrier family 23 member 2",
  "gene": "UniProtKB:Q9UGH3",
  "term_label": "L-ascorbic acid transmembrane transporter activity",
  "gene_symbol": "SLC23A2"
}